{
  "gene_symbol": "APOBEC3B",
  "gene_name": "DNA dC-dU-editing enzyme APOBEC-3B",
  "gene": "UniProtKB:Q9UH17",
  "term_label": "DNA cytosine deamination",
  "term_id": "GO:0070383"
}